phospholipase D activator activity [GO:1990583] (molecular function) References: PMID:7972129 Definition: Binds to and increases the activity of the enzyme phospholipase D. Relationships: is a type of phospholipase activator activity [GO:0016004]; positively regulates phospholipase D activity [GO:0004630]